{
  "gene_name": "Protein phosphatase 1 regulatory subunit 15A",
  "gene": "UniProtKB:O75807",
  "term_id": "GO:0000164",
  "term_label": "protein phosphatase type 1 complex",
  "gene_symbol": "PPP1R15A"
}